{
  "gene_symbol": "ZNF879",
  "term_id": "GO:0000978",
  "term_label": "RNA polymerase II cis-regulatory region sequence-specific DNA binding",
  "gene_name": "Zinc finger protein 879",
  "gene": "UniProtKB:B4DU55"
}